proboscis morphogenesis, eye-antennal disc-derived [GO:0010783] (biological process) Relationships: is a type of post-embryonic animal morphogenesis [GO:0009886]; is part of GO:0007455; is part of proboscis morphogenesis [GO:0048734] Definition: The process in which the anatomical structures of the proboscis that are derived from the eye-antennal disc are generated and organized. Sources: GOC:dph, GOC:tb